{
  "term_id": "UNKNOWN:0002",
  "gene_name": "Uncharacterized protein C7orf50",
  "gene_symbol": "C7orf50",
  "gene": "UniProtKB:Q9BRJ6",
  "term_label": "Unknown biological process"
}